furaldehyde metabolic process [GO:0033859] (biological process) Definition: The chemical reactions and pathways involving furaldehyde, a furan ring-containing aldehyde compound which can be formed from the thermal decomposition of biomass. Relationships: is a type of aldehyde metabolic process [GO:0006081] References: PMID:15338422, PMID:16652391 Sources: GOC:jp